{
  "gene_symbol": "KBTBD7",
  "gene": "UniProtKB:Q8WVZ9",
  "gene_name": "Kelch repeat and BTB domain-containing protein 7",
  "term_id": "GO:0031463",
  "term_label": "Cul3-RING ubiquitin ligase complex"
}